{
  "term_id": "GO:0005634",
  "gene_name": "Zinc finger protein 354B",
  "gene": "UniProtKB:Q96LW1",
  "term_label": "nucleus",
  "gene_symbol": "ZNF354B"
}